{
  "gene": "UniProtKB:Q96DZ5",
  "term_label": "nucleus",
  "gene_name": "CAP-Gly domain-containing linker protein 3",
  "gene_symbol": "CLIP3",
  "term_id": "GO:0005634"
}